granulocyte colony-stimulating factor binding [GO:0051916] (molecular function) Relationships: is a type of cytokine binding [GO:0019955] Definition: Binding to granulocyte colony-stimulating factor, G-CSF. Also known as: G-CSF binding, granulocyte colony stimulating factor binding Sources: GOC:ai